host thylakoid membrane [GO:0044160] (cellular component) Sources: GOC:rph Definition: The pigmented membrane of any host thylakoid. Subtypes: host cell chloroplast thylakoid membrane [GO:0033654] Relationships: is a type of host cell membrane [GO:0033644]; is a type of host cell cytoplasm part [GO:0033655]; is part of host thylakoid [GO:0044159]